{
  "gene": "UniProtKB:Q9Y4F9",
  "term_id": "UNKNOWN:0003",
  "term_label": "Unknown cellular component",
  "gene_name": "Rho family-interacting cell polarization regulator 2",
  "gene_symbol": "RIPOR2"
}